{
  "gene": "UniProtKB:Q9ULV1",
  "gene_name": "Frizzled-4",
  "term_id": "GO:0061299",
  "gene_symbol": "FZD4",
  "term_label": "retina vasculature morphogenesis in camera-type eye"
}